{
  "gene": "UniProtKB:Q8TAG9",
  "gene_name": "Exocyst complex component 6",
  "term_label": "Golgi to plasma membrane transport",
  "term_id": "GO:0006893",
  "gene_symbol": "EXOC6"
}